renal vesicle morphogenesis [GO:0072077] (biological process) Sources: GOC:mtg_kidney_jan10 Definition: The process in which the anatomical structures of the renal vesicle are generated and organized. The renal vesicle is the primordial structure of the nephron epithelium, and is formed by the condensation of mesenchymal cells. Relationships: is a type of morphogenesis of an epithelium [GO:0002009]; is part of renal vesicle development [GO:0072087]; is part of GO:0072088 Subtypes: mesonephric renal vesicle morphogenesis [GO:0061243], GO:0072283